{
  "term_id": "GO:0006400",
  "gene_name": "tRNA (guanine-N(7)-)-methyltransferase non-catalytic subunit WDR4",
  "term_label": "tRNA modification",
  "gene_symbol": "WDR4",
  "gene": "UniProtKB:P57081"
}